{
  "gene_name": "Cyclin-dependent kinase-like 3",
  "gene_symbol": "CDKL3",
  "term_label": "protein serine/threonine kinase activity",
  "term_id": "GO:0004674",
  "gene": "UniProtKB:Q8IVW4"
}